{
  "term_id": "GO:0016887",
  "term_label": "ATP hydrolysis activity",
  "gene_symbol": "OLA1",
  "gene_name": "Obg-like ATPase 1",
  "gene": "UniProtKB:Q9NTK5"
}